menstrual cycle [GO:0044850] (biological process) Definition: A type of ovulation cycle where the endometrium is shed if pregnancy does not occur. Sources: GOC:jl Relationships: is_a developmental process involved in reproduction [GO:0003006]; is a type of ovulation cycle [GO:0042698]